{
  "term_label": "ribosomal large subunit assembly",
  "gene_name": "Ribosome biogenesis protein BRX1 homolog",
  "term_id": "GO:0000027",
  "gene": "UniProtKB:Q8TDN6",
  "gene_symbol": "BRIX1"
}